{
  "term_label": "Unknown molecular function",
  "gene_symbol": "C7orf25",
  "term_id": "UNKNOWN:0001",
  "gene": "UniProtKB:Q9BPX7",
  "gene_name": "UPF0415 protein C7orf25"
}